{
  "gene_name": "Serum response factor-binding protein 1",
  "gene": "UniProtKB:Q8NEF9",
  "gene_symbol": "SRFBP1",
  "term_label": "Unknown molecular function",
  "term_id": "UNKNOWN:0001"
}